{
  "gene": "UniProtKB:P54098",
  "gene_name": "DNA polymerase subunit gamma-1",
  "term_id": "GO:0008408",
  "term_label": "3'-5' exonuclease activity",
  "gene_symbol": "POLG"
}